{
  "gene": "UniProtKB:A0A075B6U6",
  "term_id": "UNKNOWN:0001",
  "gene_name": "T cell receptor alpha variable 8-7 (pseudogene) (Fragment)",
  "term_label": "Unknown molecular function",
  "gene_symbol": "TRAV8-7"
}